{
  "gene_symbol": "KLRG2",
  "term_label": "Unknown molecular function",
  "gene_name": "Killer cell lectin-like receptor subfamily G member 2",
  "term_id": "UNKNOWN:0001",
  "gene": "UniProtKB:A4D1S0"
}